{
  "term_id": "GO:0050919",
  "term_label": "negative chemotaxis",
  "gene_name": "Semaphorin-3G",
  "gene_symbol": "SEMA3G",
  "gene": "UniProtKB:Q9NS98"
}